{
  "term_id": "GO:0000781",
  "gene_name": "5' exonuclease Apollo",
  "gene_symbol": "DCLRE1B",
  "term_label": "chromosome, telomeric region",
  "gene": "UniProtKB:Q9H816"
}